response to anoxia [GO:0034059] (biological process) Also known as: response to anoxic stress Definition: Any process that results in a change in state or activity of a cell or an organism (in terms of movement, secretion, enzyme production, gene expression, etc.) as a result of a stimulus indicating a decline in oxygen levels to trace amounts, <0.1%. Sources: GOC:kmv Subtypes: cellular response to anoxia [GO:0071454], anoxia protection [GO:0090519] Relationships: is a type of GO:0006950; is a type of response to decreased oxygen levels [GO:0036293] Note: Note that this term should not be confused with 'response to hypoxia ; GO:0001666'.